syn-stemod-13(17)-ene synthase activity [GO:0034283] (molecular function) Also known as: 9alpha-copalyl-diphosphate diphosphate-lyase [stemod-13(17)-ene-forming] activity, exo-stemodene synthase activity, stemod-13(17)-ene synthase activity, stemodene synthase activity, syn-stemodene synthase activity Definition: Catalysis of the reaction: 9-alpha-copalyl diphosphate = stemod-13(17)-ene + diphosphate. Sources: RHEA:25556 Relationships: is a type of GO:0016838